{
  "term_id": "GO:0060292",
  "gene": "UniProtKB:Q9UI40",
  "gene_symbol": "SLC24A2",
  "gene_name": "Sodium_potassium_calcium exchanger 2",
  "term_label": "long-term synaptic depression"
}